aspartate transmembrane transport [GO:0015810] (biological process) Relationships: is a type of amino acid transmembrane transport [GO:0003333]; is a type of C4-dicarboxylate transport [GO:0015740]; is a type of acidic amino acid transport [GO:0015800]; is_a GO:0071705; is a type of carboxylic acid transmembrane transport [GO:1905039] Also known as: aspartate transport, mitochondrial aspartate/glutamate transport Subtypes: D-aspartate transmembrane transport [GO:0070777], L-aspartate transmembrane transport [GO:0070778], GO:0090453 Sources: GOC:go_curators, ISBN:0198506732 Definition: The process in which aspartate is transported across a lipid bilayer, from one side of a membrane to the other.